{
  "gene_name": "Elongin-C",
  "term_label": "protein-macromolecule adaptor activity",
  "gene_symbol": "ELOC",
  "gene": "UniProtKB:Q15369",
  "term_id": "GO:0030674"
}